{
  "gene": "UniProtKB:Q9H422",
  "term_label": "Unknown biological process",
  "gene_name": "Homeodomain-interacting protein kinase 3",
  "term_id": "UNKNOWN:0002",
  "gene_symbol": "HIPK3"
}